{
  "gene_symbol": "KRTAP6-3",
  "gene": "UniProtKB:Q3LI67",
  "term_id": "UNKNOWN:0001",
  "gene_name": "Keratin-associated protein 6-3",
  "term_label": "Unknown molecular function"
}